{
  "gene_symbol": "TRBJ1-1",
  "gene": "UniProtKB:A0A0J9YXA8",
  "gene_name": "T cell receptor beta joining 1-1",
  "term_label": "Unknown biological process",
  "term_id": "UNKNOWN:0002"
}